{
  "term_id": "UNKNOWN:0003",
  "gene": "UniProtKB:Q6ZUS6",
  "gene_name": "Coiled-coil domain-containing protein 149",
  "term_label": "Unknown cellular component",
  "gene_symbol": "CCDC149"
}